cellular response to pH [GO:0071467] (biological process) Sources: GOC:mah, Wikipedia:PH Subtypes: GO:0036244, cellular response to acidic pH [GO:0071468], cellular response to alkaline pH [GO:0071469] Relationships: is a type of response to pH [GO:0009268]; is_a cellular response to abiotic stimulus [GO:0071214] Definition: Any process that results in a change in state or activity of a cell (in terms of movement, secretion, enzyme production, gene expression, etc.) as a result of a pH stimulus. pH is a measure of the acidity or basicity of an aqueous solution.